cytosolic transport [GO:0016482] (biological process) Subtypes: Golgi to endosome transport [GO:0006895], retrograde transport, endosome to Golgi [GO:0042147], vesicle-mediated cholesterol transport [GO:0090119], Golgi to lysosome transport [GO:0090160], GO:1901950, plastid to vacuole vesicle-mediated transport [GO:1904962] Relationships: is a type of GO:0046907; occurs in cytosol [GO:0005829] Definition: The directed movement of substances or organelles within the cytosol. Sources: GOC:ai